{
  "gene_symbol": "H2BC18",
  "gene_name": "Histone H2B type 2-F",
  "term_id": "GO:0061844",
  "gene": "UniProtKB:Q5QNW6",
  "term_label": "antimicrobial humoral immune response mediated by antimicrobial peptide"
}